{
  "gene_name": "Homeobox protein Nkx-2.2",
  "term_id": "GO:0005634",
  "term_label": "nucleus",
  "gene": "UniProtKB:O95096",
  "gene_symbol": "NKX2-2"
}